{
  "gene_name": "Coiled-coil domain-containing protein 74A",
  "gene_symbol": "CCDC74A",
  "term_label": "Unknown molecular function",
  "gene": "UniProtKB:Q96AQ1",
  "term_id": "UNKNOWN:0001"
}